RNA strand annealing activity [GO:0033592] (molecular function) Relationships: is a type of single-stranded RNA binding [GO:0003727]; is a type of catalytic activity, acting on RNA [GO:0140098]; is a type of annealing activity [GO:0140666] References: PMID:7543843 Sources: GOC:mah Definition: An activity that facilitates the formation of a complementary double-stranded RNA molecule.